{
  "gene": "UniProtKB:A4D256",
  "gene_name": "Dual specificity protein phosphatase CDC14C",
  "term_label": "spindle pole",
  "term_id": "GO:0000922",
  "gene_symbol": "CDC14C"
}